{
  "term_label": "Unknown molecular function",
  "gene_name": "Uncharacterized protein C16orf96",
  "term_id": "UNKNOWN:0001",
  "gene_symbol": "C16orf96",
  "gene": "UniProtKB:A6NNT2"
}